{
  "term_label": "regulation of neuronal synaptic plasticity",
  "gene_symbol": "CAMK2D",
  "term_id": "GO:0048168",
  "gene_name": "Calcium_calmodulin-dependent protein kinase type II subunit delta",
  "gene": "UniProtKB:Q13557"
}